{
  "gene": "UniProtKB:Q9NR48",
  "gene_symbol": "ASH1L",
  "term_label": "regulation of DNA-templated transcription",
  "term_id": "GO:0006355",
  "gene_name": "Histone-lysine N-methyltransferase ASH1L"
}